{
  "gene_symbol": "CS",
  "term_id": "GO:0005975",
  "term_label": "carbohydrate metabolic process",
  "gene": "UniProtKB:O75390",
  "gene_name": "Citrate synthase, mitochondrial"
}